{
  "gene_name": "Transcription factor SOX-9",
  "gene_symbol": "SOX9",
  "term_label": "nucleus",
  "gene": "UniProtKB:P48436",
  "term_id": "GO:0005634"
}